{
  "gene": "UniProtKB:Q86VZ5",
  "term_label": "plasma membrane",
  "gene_symbol": "SGMS1",
  "gene_name": "Phosphatidylcholine:ceramide cholinephosphotransferase 1",
  "term_id": "GO:0005886"
}